symbiont-mediated perturbation of host actin cytoskeleton via filamentous actin depolymerization [GO:0141030] (biological process) Definition: The process in which an organism effects a change that impairs the structure or function of the host actin cytoskeleton by depolymerizing the host filamentous actin. The host is defined as the larger of the organisms involved in a symbiotic interaction. Relationships: is a type of symbiont-mediated perturbation of host actin cytoskeleton [GO:0141027] References: PMID:11889090, PMID:28800062